histone H3S57 kinase activity [GO:0140855] (molecular function) Relationships: is a type of protein serine/threonine kinase activity [GO:0004674]; is a type of histone H3 kinase activity [GO:0140996] References: PMID:24820035 Definition: Catalysis of the reaction: histone H3-serine (position 57) + ATP = histone H3-phosphoserine (position 57) + ADP. This reaction is the addition of a phosphate group to the serine residue at position 57 of histone H3. Note: Comment: Note that the residue position corresponds to the canonical human H3 histone (UniProtKB:P84243); this residue is conserved across all eukaryotes. Residue 1 is the first residue following removal of the initiating Methionine (Met). Note that each histone is encoded by multiple genes, and sequences may vary across different genes within an organism. Also known as: histone kinase activity (H3-S57 specific), histone serine kinase activity (H3-S57 specific), histone-serine kinase activity (H3-S57 specific)